{
  "term_label": "RNA polymerase II cis-regulatory region sequence-specific DNA binding",
  "gene_symbol": "MXD1",
  "gene_name": "Max dimerization protein 1",
  "gene": "UniProtKB:Q05195",
  "term_id": "GO:0000978"
}